glycolytic process [GO:0006096] (BP) Definition: The chemical reactions and pathways resulting in the breakdown of a carbohydrate into pyruvate, with the concomitant production of a small amount of ATP and the reduction of NAD(P) to NAD(P)H. Glycolysis begins with the metabolism of a carbohydrate to generate products that can enter the pathway and ends with the production of pyruvate. Pyruvate may be converted to acetyl-coenzyme A, ethanol, lactate, or other small molecules. Relationships: is a type of pyruvate metabolic process [GO:0006090]; is a type of GO:0006091; is a type of carbohydrate catabolic process [GO:0016052]; is a type of pyridine nucleotide catabolic process [GO:0019364]; is a type of ADP catabolic process [GO:0046032]; is a type of ATP metabolic process [GO:0046034]; is a type of nicotinamide nucleotide metabolic process [GO:0046496]; is part of aerobic respiration [GO:0009060]; has part GO:0004618; has part phosphoglycerate mutase activity [GO:0004619]; has part phosphopyruvate hydratase activity [GO:0004634]; BFO_0000051 pyruvate kinase activity [GO:0004743]; has part glyceraldehyde-3-phosphate dehydrogenase [NAD(P)+] (phosphorylating) activity [GO:0043891] Also known as: Embden-Meyerhof pathway, Embden-Meyerhof-Parnas pathway, anaerobic glycolysis, glycolysis, modified Embden-Meyerhof pathway Sources: GOC:bf, GOC:dph, ISBN:0201090910, ISBN:0716720094, ISBN:0879010479 Subtypes: GO:0061613, glycolytic process through fructose-6-phosphate [GO:0061615], glycolytic process through fructose-1-phosphate [GO:0061625], glycolytic process via Entner-Doudoroff Pathway [GO:0061688], glycolytic process from sucrose [GO:0061704] Regulation: RO_0002211 by regulation of glycolytic process [GO:0006110]; RO_0002212 by negative regulation of glycolytic process [GO:0045820]; positively regulated by positive regulation of glycolytic process [GO:0045821]